{
  "gene_symbol": "MEIS2",
  "gene_name": "Homeobox protein Meis2",
  "term_label": "embryonic pattern specification",
  "gene": "UniProtKB:O14770",
  "term_id": "GO:0009880"
}